{
  "gene": "UniProtKB:P06454",
  "term_label": "positive regulation of transcription by RNA polymerase II",
  "term_id": "GO:0045944",
  "gene_name": "Prothymosin alpha",
  "gene_symbol": "PTMA"
}